B cell receptor signaling pathway [GO:0050853] (biological process) Sources: GOC:add Definition: The series of molecular signals initiated by the cross-linking of an antigen receptor on a B cell. Also known as: B cell receptor signalling pathway, B lymphocyte receptor signaling pathway, B lymphocyte receptor signalling pathway, B-cell receptor signaling pathway, B-cell receptor signalling pathway, B-lymphocyte receptor signaling pathway, B-lymphocyte receptor signalling pathway Relationships: is a type of GO:0050851 Subtypes: B cell receptor apoptotic signaling pathway [GO:1990117] Regulation: regulated by GO:0050855; negatively regulated by GO:0050859; positively regulated by GO:0050861